{
  "gene_name": "Sorting nexin-12",
  "gene": "UniProtKB:Q9UMY4",
  "term_label": "early endosome membrane",
  "gene_symbol": "SNX12",
  "term_id": "GO:0031901"
}